age-related resistance [GO:0090644] (biological process) References: PMID:17635216, PMID:19694953 Regulation: regulated by regulation of age-related resistance [GO:1904248]; RO_0002212 by negative regulation of age-related resistance [GO:1904249]; positively regulated by positive regulation of age-related resistance [GO:1904250] Definition: An innate immune response that is positively correlated with host plant development. As a plant develops, its innate resistance to pathogenic infections increases. The mechanisms involved in age-related resistance differ in nature or in aspects of regulation from the hypersensitive response (HR), systemic acquired resistance (SAR), or induced systemic resistance (ISR). Also known as: developmental resistance, ontogenic resistance, ARR, adult seedling resistance, flowering-induced resistance, mature seedling resistance, senescence-induced resistance Relationships: is a type of developmental process [GO:0032502]; is a type of innate immune response [GO:0045087]